{
  "gene": "UniProtKB:Q04844",
  "term_label": "synapse",
  "term_id": "GO:0045202",
  "gene_symbol": "CHRNE",
  "gene_name": "Acetylcholine receptor subunit epsilon"
}